{
  "gene_name": "Putative guanine nucleotide-binding protein G(I)_G(S)_G(O) subunit gamma-14",
  "term_label": "G protein-coupled receptor signaling pathway",
  "gene_symbol": "GNG14",
  "gene": "UniProtKB:A0A1W2PPG7",
  "term_id": "GO:0007186"
}